{
  "gene_symbol": "C9orf72",
  "term_id": "UNKNOWN:0001",
  "term_label": "Unknown molecular function",
  "gene_name": "Guanine nucleotide exchange factor C9orf72",
  "gene": "UniProtKB:Q96LT7"
}